D-lactate dehydrogenase (cytochrome c-553) activity [GO:0047051] (molecular function) Also known as: (R)-lactate:ferricytochrome-c-553 2-oxidoreductase activity Relationships: is a type of oxidoreductase activity, acting on the CH-OH group of donors, cytochrome as acceptor [GO:0016898] Sources: RHEA:16465 Definition: Catalysis of the reaction: (R)-lactate + 2 [Fe(III)cytochrome c553] = 2 [Fe(II)cytochrome c553] + 2 H+ + pyruvate.